{
  "gene_symbol": "MTF1",
  "term_label": "RNA polymerase II cis-regulatory region sequence-specific DNA binding",
  "gene_name": "Metal regulatory transcription factor 1",
  "gene": "UniProtKB:Q14872",
  "term_id": "GO:0000978"
}